{
  "term_id": "UNKNOWN:0003",
  "term_label": "Unknown cellular component",
  "gene": "UniProtKB:Q0D2K5",
  "gene_name": "Putative EGF-like and EMI domain-containing protein 1",
  "gene_symbol": "EGFEM1P"
}